steroid-lactonase activity [GO:0050293] (molecular function) Definition: Catalysis of the reaction: H2O + testololactone = H+ + testolate. Also known as: testololactone lactonohydrolase activity Relationships: is a type of GO:0052689 Sources: EC:3.1.1.37, RHEA:13721